{
  "term_label": "cytoplasmic stress granule",
  "gene": "UniProtKB:Q9H361",
  "gene_name": "Polyadenylate-binding protein 3",
  "term_id": "GO:0010494",
  "gene_symbol": "PABPC3"
}